{
  "term_label": "protein serine/threonine kinase activity",
  "gene": "UniProtKB:Q9P0L2",
  "gene_name": "Serine_threonine-protein kinase MARK1",
  "term_id": "GO:0004674",
  "gene_symbol": "MARK1"
}